{
  "term_label": "Unknown molecular function",
  "gene_symbol": "NDUFAF4",
  "gene": "UniProtKB:Q9P032",
  "gene_name": "NADH dehydrogenase [ubiquinone] 1 alpha subcomplex assembly factor 4",
  "term_id": "UNKNOWN:0001"
}